{
  "gene_name": "Immortalization up-regulated protein",
  "gene": "UniProtKB:Q9GZP8",
  "gene_symbol": "IMUP",
  "term_label": "Unknown molecular function",
  "term_id": "UNKNOWN:0001"
}